{
  "gene": "UniProtKB:O15105",
  "term_id": "GO:0060395",
  "gene_symbol": "SMAD7",
  "gene_name": "Mothers against decapentaplegic homolog 7",
  "term_label": "SMAD protein signal transduction"
}